{
  "gene": "UniProtKB:Q7Z7G2",
  "gene_symbol": "CPLX4",
  "term_id": "GO:0031630",
  "term_label": "regulation of synaptic vesicle fusion to presynaptic active zone membrane",
  "gene_name": "Complexin-4"
}